effector-mediated suppression of host pattern-triggered immunity [GO:0052034] (biological process) Relationships: is a type of effector-mediated suppression of host innate immune response [GO:0140403] Also known as: negative regulation by organism of pathogen-associated molecular pattern-induced innate immune response of other organism involved in symbiotic interaction, suppression by symbiont of microbe-associated molecular pattern-induced host innate immune response, down regulation by symbiont of pathogen-associated molecular pattern-induced host innate immunity, down-regulation by symbiont of pathogen-associated molecular pattern-induced host innate immunity, downregulation by symbiont of pathogen-associated molecular pattern-induced host innate immunity, inhibition by symbiont of pathogen-associated molecular pattern-induced host innate immunity, negative regulation by symbiont of microbe-associated molecular pattern-induced host innate immune response, negative regulation by symbiont of microbe-associated molecular pattern-induced host innate immunity, suppression of MAMP induced host innate immunity, suppression of MAMP-induced host innate immunity, suppression of PAMP induced host innate immunity, suppression of PAMP-induced host innate immunity, suppression of general elicitor induced host innate immunity, suppression of general elicitor-induced host innate immunity, suppression of pathogen-associated molecular pattern-induced host innate immunity Definition: A process mediated by a molecule secreted by a symbiont that results in the suppression of the innate immune response of the host organism via recognition of a microbe-associated molecular pattern. The innate immune response is the host's first line of defense against infection. The host is defined as the larger of the organisms involved in a symbiotic interaction. Sources: GOC:mah Subtypes: effector-mediated suppression of host pattern-triggered immunity signaling [GO:0140423]